{
  "gene_symbol": "PCDHGC3",
  "term_label": "cell adhesion",
  "term_id": "GO:0007155",
  "gene_name": "Protocadherin gamma-C3",
  "gene": "UniProtKB:Q9UN70"
}